{
  "gene_symbol": "CROCCP2",
  "gene_name": "Putative ciliary rootlet coiled-coil protein-like 1 protein",
  "term_label": "Unknown cellular component",
  "term_id": "UNKNOWN:0003",
  "gene": "UniProtKB:Q86T23"
}